{
  "gene": "UniProtKB:P06746",
  "term_label": "nucleus",
  "term_id": "GO:0005634",
  "gene_symbol": "POLB",
  "gene_name": "DNA polymerase beta"
}